contractile ring [GO:0070938] (cellular component) Subtypes: actomyosin contractile ring [GO:0005826] Also known as: constriction ring, cytokinetic ring Definition: A cytoskeletal structure composed of filamentous protein that forms beneath the membrane of many cells or organelles, in the plane of cell or organelle division. Ring contraction is associated with centripetal growth of the membrane that divides the cytoplasm of the two daughter cells or organelles. References: PMID:10791428, PMID:17913889 Sources: GOC:mah, ISBN:0123645859, ISBN:0792354923 Relationships: is a type of cellular anatomical structure [GO:0110165]